{
  "gene_symbol": "OR2A1",
  "gene_name": "Olfactory receptor 2A1_2A42",
  "gene": "UniProtKB:Q8NGT9",
  "term_label": "olfactory receptor activity",
  "term_id": "GO:0004984"
}